{
  "gene_symbol": "SMIM6",
  "gene_name": "Small integral membrane protein 6",
  "gene": "UniProtKB:P0DI80",
  "term_label": "Unknown cellular component",
  "term_id": "UNKNOWN:0003"
}